helper T cell enhancement of T cell mediated immune response [GO:0035398] (biological process) Definition: Positive regulation of a T cell mediated immune response mediated via cytokine production by a helper T cell. Sources: GOC:add Also known as: helper T cell enhancement of T cell mediated immunity, provision of T cell help to T cell Relationships: is a type of positive regulation of T cell mediated immunity [GO:0002711]; is a type of helper T cell enhancement of adaptive immune response [GO:0035397]